{
  "gene": "UniProtKB:A0A0K0K1E9",
  "term_id": "UNKNOWN:0001",
  "gene_name": "T cell receptor beta variable 7-7",
  "term_label": "Unknown molecular function",
  "gene_symbol": "TRBV7-7"
}